{
  "gene_name": "Lymphocyte antigen 6L",
  "gene": "UniProtKB:H3BQJ8",
  "term_label": "Unknown molecular function",
  "term_id": "UNKNOWN:0001",
  "gene_symbol": "LY6L"
}